regulation of cell integrity MAPK cascade [GO:1903137] (biological process) Also known as: regulation of MAPK cascade involved in cell wall organization or biogenesis, regulation of MAPKKK cascade involved in cell wall biogenesis, regulation of cell integrity MAPK pathway, regulation of cell wall biogenesis, MAPKKK cascade, regulation of MAPK cascade involved in cell wall biogenesis, regulation of Mpk1 cascade, regulation of PMK1-MAPK signal transduction pathway, regulation of Pmk1 MAPK cell integrity signaling, regulation of Pmk1 mitogen-activated protein kinase (MAPK) cell integrity pathway, regulation of Slt2 cascade, regulation of cell wall integrity MAPK cascade Sources: GOC:vw Definition: Any process that modulates the frequency, rate or extent of a cell integrity MAPK cascade. Relationships: is a type of GO:0032872; regulates cell integrity MAPK cascade [GO:0000196] Subtypes: negative regulation of cell integrity MAPK cascade [GO:1903138], positive regulation of cell integrity MAPK cascade [GO:1903139]